anandamide 14,15 epoxidase activity [GO:0062189] (molecular function) Definition: Catalysis of the reaction: N-(5Z,8Z,11Z,14Z-eicosatetraenoyl)-ethanolamine + O2 + reduced [NADPH--hemoprotein reductase] = H+ + H2O + N-(14,15-epoxy-5Z,8Z,11Z-eicosatrienoyl)-ethanolamine + oxidized [NADPH--hemoprotein reductase]. References: PMID:21289075 Sources: RHEA:53148 Relationships: is a type of anandamide epoxidase activity [GO:0062186]